{
  "term_label": "brush border",
  "term_id": "GO:0005903",
  "gene": "UniProtKB:Q8N130",
  "gene_symbol": "SLC34A3",
  "gene_name": "Sodium-dependent phosphate transport protein 2C"
}